{
  "gene": "UniProtKB:Q13021",
  "gene_symbol": "MALL",
  "gene_name": "MAL-like protein",
  "term_id": "GO:0016020",
  "term_label": "membrane"
}